{
  "gene": "UniProtKB:Q96S59",
  "term_label": "proteasome-mediated ubiquitin-dependent protein catabolic process",
  "gene_name": "Ran-binding protein 9",
  "gene_symbol": "RANBP9",
  "term_id": "GO:0043161"
}